biosynthetic process of antibacterial peptides active against Gram-negative bacteria [GO:0002812] (biological process) Relationships: is a type of antibacterial peptide biosynthetic process [GO:0002780]; is part of defense response to Gram-negative bacterium [GO:0050829] Definition: The chemical reactions and pathways resulting in the formation of an antibacterial peptide with activity against Gram-negative bacteria. References: PMID:11807545 Sources: GOC:add Regulation: regulated by GO:0002813; negatively regulated by negative regulation of biosynthetic process of antibacterial peptides active against Gram-negative bacteria [GO:0002814]; positively regulated by positive regulation of biosynthetic process of antibacterial peptides active against Gram-negative bacteria [GO:0006964]